extrinsic component of stromal side of plastid inner membrane [GO:0035454] (cellular component) Also known as: extrinsic to stromal leaflet of plastid inner membrane, peripheral to stromal side of plastid inner membrane, extrinsic to stromal side of plastid inner membrane Relationships: is a type of extrinsic component of lumenal side of plastid thylakoid membrane [GO:0035450] Definition: The component of a plastid inner membrane consisting of gene products and protein complexes that are loosely bound to its stromal surface, but not integrated into the hydrophobic region. Sources: GOC:bf, GOC:dos